{
  "term_label": "regulation of transcription by RNA polymerase II",
  "gene_name": "Cyclic AMP-dependent transcription factor ATF-7",
  "gene": "UniProtKB:P17544",
  "term_id": "GO:0006357",
  "gene_symbol": "ATF7"
}